{
  "gene": "UniProtKB:Q9Y6H5",
  "gene_symbol": "SNCAIP",
  "term_id": "UNKNOWN:0002",
  "gene_name": "Synphilin-1",
  "term_label": "Unknown biological process"
}